{
  "gene": "UniProtKB:P01031",
  "term_label": "Unknown molecular function",
  "gene_symbol": "C5",
  "term_id": "UNKNOWN:0001",
  "gene_name": "Complement C5"
}